{
  "gene": "UniProtKB:Q8N4F0",
  "gene_name": "BPI fold-containing family B member 2",
  "term_label": "Unknown biological process",
  "term_id": "UNKNOWN:0002",
  "gene_symbol": "BPIFB2"
}